{
  "gene_symbol": "KLKB1",
  "gene_name": "Plasma kallikrein",
  "gene": "UniProtKB:P03952",
  "term_label": "serine-type peptidase activity",
  "term_id": "GO:0008236"
}